{
  "term_id": "GO:0032963",
  "gene_name": "Prolyl 3-hydroxylase 3",
  "gene": "UniProtKB:Q8IVL6",
  "gene_symbol": "P3H3",
  "term_label": "collagen metabolic process"
}